intracellularly phosphatidylinositol-3,5-bisphosphate-gated monatomic cation channel activity [GO:0097682] (molecular function) Definition: Enables the transmembrane transfer of cations by a channel that opens when phosphatidylinositol-3,5-bisphosphate has been bound by the channel complex or one of its constituent parts. Also known as: intracellular phosphatidylinositol-3,5-bisphosphate-sensitive cation channel activity, intracellular phosphatidylinositol-3,5-bisphosphate-sensitive monatomic cation channel activity References: PMID:24375408 Sources: GOC:ha Relationships: is a type of GO:0005217; is a type of ligand-gated monoatomic cation channel activity [GO:0099094]